{
  "gene_symbol": "TAFA5",
  "term_label": "receptor ligand activity",
  "term_id": "GO:0048018",
  "gene_name": "Chemokine-like protein TAFA-5",
  "gene": "UniProtKB:Q7Z5A7"
}